dorsal/ventral neural tube patterning [GO:0021904] (biological process) References: PMID:11262869 Sources: GOC:cls, GOC:dgh, GOC:dph, GOC:jid, GO_REF:0000021 Relationships: is a type of GO:0009953; is part of neural tube patterning [GO:0021532] Definition: The process in which the neural tube is regionalized in the dorsoventral axis. Also known as: dorsal-ventral neural tube patterning, dorsoventral neural tube patterning